glycine N-choloyltransferase activity [GO:0047963] (MF) Definition: Catalysis of the reaction: choloyl-CoA + glycine = CoA + glycocholate. Also known as: BACAT activity, BAT activity, amino acid N-choloyltransferase activity, bile acid-CoA:amino acid N-acyltransferase activity, choloyl-CoA:glycine N-choloyltransferase activity, cholyl-CoA glycine-taurine N-acyltransferase activity, cholyl-CoA:taurine N-acyltransferase activity, glycine--taurine N-acyltransferase activity Relationships: is a type of acyltransferase activity, transferring groups other than amino-acyl groups [GO:0016747] Sources: EC:2.3.1.65, MetaCyc:GLYCINE-N-CHOLOYLTRANSFERASE-RXN